{
  "term_id": "UNKNOWN:0001",
  "gene_symbol": "RD3",
  "gene_name": "Protein RD3",
  "gene": "UniProtKB:Q7Z3Z2",
  "term_label": "Unknown molecular function"
}